{
  "gene": "UniProtKB:Q01534",
  "term_label": "chromatin binding",
  "gene_symbol": "TSPY1",
  "gene_name": "Testis-specific Y-encoded protein 1",
  "term_id": "GO:0003682"
}